{
  "term_label": "hormone biosynthetic process",
  "gene_symbol": "CYP17A1",
  "gene": "UniProtKB:P05093",
  "term_id": "GO:0042446",
  "gene_name": "Steroid 17-alpha-hydroxylase_17,20 lyase"
}